{
  "gene": "UniProtKB:Q9Y484",
  "gene_symbol": "WDR45",
  "gene_name": "WD repeat domain phosphoinositide-interacting protein 4",
  "term_label": "phagophore assembly site membrane",
  "term_id": "GO:0034045"
}